poly(glycerol-phosphate) alpha-glucosyltransferase activity [GO:0047265] (molecular function) Definition: Catalysis of the reaction: poly(glycerol phosphate) + UDP-D-glucose = alpha-D-glucosylpoly(glycerol phosphate) + UDP. Sources: EC:2.4.1.52 Also known as: UDP glucose-poly(glycerol-phosphate) alpha-glucosyltransferase activity, UDP-glucose:poly(glycerol-phosphate) alpha-D-glucosyltransferase activity, UDPglucose:poly(glycerol-phosphate) alpha-D-glucosyltransferase activity, uridine diphosphoglucose-poly(glycerol-phosphate) alpha-glucosyltransferase activity Relationships: is a type of UDP-glucosyltransferase activity [GO:0035251]